{
  "term_id": "GO:0000298",
  "gene": "UniProtKB:Q9NZJ9",
  "gene_symbol": "NUDT4",
  "gene_name": "Diphosphoinositol polyphosphate phosphohydrolase 2",
  "term_label": "endopolyphosphatase activity"
}